{
  "gene_name": "Origin recognition complex subunit 4",
  "term_id": "GO:0006270",
  "gene": "UniProtKB:O43929",
  "term_label": "DNA replication initiation",
  "gene_symbol": "ORC4"
}